nuclear thyroid hormone receptor binding [GO:0046966] (molecular function) Also known as: thyroid hormone receptor binding, ligand-dependent thyroid hormone receptor interactor activity Definition: Binding to a nuclear thyroid hormone receptor. Sources: GOC:ai Relationships: is a type of nuclear receptor binding [GO:0016922]